{
  "term_id": "GO:0030593",
  "gene": "UniProtKB:P02776",
  "gene_symbol": "PF4",
  "term_label": "neutrophil chemotaxis",
  "gene_name": "Platelet factor 4"
}